{
  "term_id": "GO:0006355",
  "gene_name": "Non-POU domain-containing octamer-binding protein",
  "gene": "UniProtKB:Q15233",
  "term_label": "regulation of DNA-templated transcription",
  "gene_symbol": "NONO"
}